{
  "gene": "UniProtKB:A6NFA1",
  "term_id": "GO:0017147",
  "gene_symbol": "TRABD2B",
  "term_label": "Wnt-protein binding",
  "gene_name": "Metalloprotease TIKI2"
}